{
  "gene_symbol": "IGSF9B",
  "term_label": "Unknown biological process",
  "gene_name": "Protein turtle homolog B",
  "term_id": "UNKNOWN:0002",
  "gene": "UniProtKB:Q9UPX0"
}